{
  "gene_symbol": "CEBPD",
  "gene_name": "CCAAT_enhancer-binding protein delta",
  "term_id": "GO:0000981",
  "gene": "UniProtKB:P49716",
  "term_label": "DNA-binding transcription factor activity, RNA polymerase II-specific"
}